{
  "gene_symbol": "AP3D1",
  "gene": "UniProtKB:O14617",
  "term_id": "GO:0098943",
  "gene_name": "AP-3 complex subunit delta-1",
  "term_label": "neurotransmitter receptor transport, postsynaptic endosome to lysosome"
}